{
  "term_id": "GO:0007165",
  "gene": "UniProtKB:Q5VSY0",
  "term_label": "signal transduction",
  "gene_symbol": "GKAP1",
  "gene_name": "G kinase-anchoring protein 1"
}